{
  "gene_symbol": "PLA2G2E",
  "gene_name": "Group IIE secretory phospholipase A2",
  "term_id": "UNKNOWN:0003",
  "term_label": "Unknown cellular component",
  "gene": "UniProtKB:Q9NZK7"
}